{
  "term_id": "GO:0051015",
  "gene_symbol": "MYO1A",
  "term_label": "actin filament binding",
  "gene": "UniProtKB:Q9UBC5",
  "gene_name": "Unconventional myosin-Ia"
}